{
  "gene": "UniProtKB:Q8N139",
  "gene_symbol": "ABCA6",
  "term_id": "UNKNOWN:0003",
  "term_label": "Unknown cellular component",
  "gene_name": "ATP-binding cassette sub-family A member 6"
}